{
  "term_id": "UNKNOWN:0001",
  "gene_name": "Putative protein FAM10A5",
  "gene_symbol": "ST13P5",
  "gene": "UniProtKB:Q8NFI4",
  "term_label": "Unknown molecular function"
}